{
  "term_label": "Unknown biological process",
  "gene": "UniProtKB:A0A1B0GTI1",
  "term_id": "UNKNOWN:0002",
  "gene_symbol": "CCDC201",
  "gene_name": "Coiled-coil domain-containing protein 201"
}